mannan 1,4-mannobiosidase activity [GO:0033928] (molecular function) Also known as: 1,4-beta-D-mannan mannobiohydrolase activity, exo-1,4-beta-mannobiohydrolase activity, exo-beta-mannanase activity, mannan 1,4-beta-mannobiosidase activity Relationships: is a type of hydrolase activity, hydrolyzing O-glycosyl compounds [GO:0004553] Sources: EC:3.2.1.100 Definition: Catalysis of the hydrolysis of (1->4)-beta-D-mannosidic linkages in (1->4)-beta-D-mannans, to remove successive mannobiose residues from the non-reducing chain ends.